{
  "gene_symbol": "TP53",
  "term_label": "nucleus",
  "term_id": "GO:0005634",
  "gene": "UniProtKB:P04637",
  "gene_name": "Cellular tumor antigen p53"
}